{
  "gene_symbol": "ZFYVE1",
  "term_id": "GO:0140042",
  "gene": "UniProtKB:Q9HBF4",
  "gene_name": "Zinc finger FYVE domain-containing protein 1",
  "term_label": "lipid droplet formation"
}